{
  "gene_name": "T-cell surface glycoprotein CD1e, membrane-associated",
  "gene": "UniProtKB:P15812",
  "gene_symbol": "CD1E",
  "term_label": "antigen processing and presentation, exogenous lipid antigen via MHC class Ib",
  "term_id": "GO:0048007"
}